{
  "term_id": "UNKNOWN:0002",
  "gene_name": "Transmembrane protein 200B",
  "gene_symbol": "TMEM200B",
  "gene": "UniProtKB:Q69YZ2",
  "term_label": "Unknown biological process"
}